{
  "term_label": "nucleus",
  "gene_name": "NEDD4-binding protein 1",
  "gene": "UniProtKB:O75113",
  "gene_symbol": "N4BP1",
  "term_id": "GO:0005634"
}